{
  "gene_symbol": "A8MWL6",
  "term_id": "GO:0030672",
  "gene_name": "Putative synaptogyrin-2 like protein",
  "gene": "UniProtKB:A8MWL6",
  "term_label": "synaptic vesicle membrane"
}